{
  "term_id": "UNKNOWN:0001",
  "gene": "UniProtKB:Q8NEA9",
  "gene_symbol": "GMCL2",
  "term_label": "Unknown molecular function",
  "gene_name": "Germ cell-less protein-like 2"
}